{
  "term_id": "GO:0005543",
  "gene_symbol": "NUP35",
  "term_label": "phospholipid binding",
  "gene": "UniProtKB:Q8NFH5",
  "gene_name": "Nucleoporin NUP35"
}